{
  "gene": "UniProtKB:Q93096",
  "gene_symbol": "PTP4A1",
  "term_label": "protein tyrosine phosphatase activity",
  "gene_name": "Protein tyrosine phosphatase type IVA 1",
  "term_id": "GO:0004725"
}